{
  "gene_symbol": "EXOG",
  "term_id": "GO:0008409",
  "gene_name": "Nuclease EXOG, mitochondrial",
  "term_label": "5'-3' exonuclease activity",
  "gene": "UniProtKB:Q9Y2C4"
}